{
  "term_id": "UNKNOWN:0001",
  "gene": "UniProtKB:O60220",
  "gene_name": "Mitochondrial import inner membrane translocase subunit Tim8 A",
  "term_label": "Unknown molecular function",
  "gene_symbol": "TIMM8A"
}